adenylate cyclase-activating glucose-activated G protein-coupled receptor signaling pathway [GO:0010619] (biological process) Also known as: activation of adenylate cyclase activity by glucose involved in G-protein signaling, activation of adenylate cyclase activity by glucose-triggered G-protein signaling pathway, activation of adenylate cyclase activity by glucose-triggered G-protein signalling pathway, glucose-sensing PKA pathway Sources: GOC:dph, GOC:signaling, GOC:tb Relationships: is a type of adenylate cyclase-activating G protein-coupled receptor signaling pathway [GO:0007189]; is part of glucose mediated signaling pathway [GO:0010255] Definition: An adenylate cyclase-activating G protein-coupled receptor signaling pathway initiated by glucose binding to its receptor on the surface of the target cell, and ending with the regulation of a downstream cellular process. Regulation: regulated by regulation of adenylate cyclase-activating glucose-activated G protein-coupled receptor signaling pathway [GO:0110033]; negatively regulated by negative regulation of adenylate cyclase-activating glucose-activated G protein-coupled receptor signaling pathway [GO:0110034]